Golgi to secretory granule transport [GO:0055107] (BP) Relationships: is_a intracellular transport [GO:0046907] Sources: GOC:curators Definition: The directed movement of proteins from the Golgi to a secretory granule. The secretory granule is a membrane-bounded particle, usually protein, formed in the granular endoplasmic reticulum and the Golgi complex.